{
  "gene_symbol": "C1RL",
  "term_id": "GO:0031638",
  "gene": "UniProtKB:Q9NZP8",
  "gene_name": "Complement C1r subcomponent-like protein",
  "term_label": "zymogen activation"
}